23S rRNA pseudouridine(1911/1915/1917) synthase activity [GO:0160140] (molecular function) Sources: EC:5.4.99.23, RHEA:42524 Definition: Catalysis of the reaction: uridine(1911/1915/1917) in 23S rRNA = pseudouridine(1911/1915/1917) in 23S rRNA. Relationships: is a type of GO:0120159